regulation of mitotic spindle disassembly [GO:1904686] (biological process) Relationships: is a type of regulation of mitotic spindle organization [GO:0060236]; regulates mitotic spindle disassembly [GO:0051228] Definition: Any process that modulates the frequency, rate or extent of mitotic spindle disassembly. References: PMID:25963819 Sources: GOC:TermGenie, GO_REF:0000058 Subtypes: positive regulation of mitotic spindle disassembly [GO:1904687] Also known as: regulation of mitotic spindle breakdown, regulation of mitotic spindle catabolism, regulation of mitotic spindle degradation, regulation of spindle breakdown during mitosis, regulation of spindle degradation during mitosis, regulation of spindle disassembly during mitosis